{
  "gene_name": "N-acetylglucosaminyl-phosphatidylinositol de-N-acetylase",
  "gene": "UniProtKB:Q9Y2B2",
  "term_label": "Unknown biological process",
  "term_id": "UNKNOWN:0002",
  "gene_symbol": "PIGL"
}